{
  "term_id": "GO:0000398",
  "gene_name": "Pre-mRNA-splicing factor CWC22 homolog",
  "gene_symbol": "CWC22",
  "gene": "UniProtKB:Q9HCG8",
  "term_label": "mRNA splicing, via spliceosome"
}